sulfur compound transport [GO:0072348] (biological process) Subtypes: GO:0000101, GO:0000316, thiosulfate transport [GO:0015709], nucleotide-sulfate transport [GO:0015715], S-adenosyl-L-methionine transport [GO:0015805], S-methylmethionine transport [GO:0015806], biotin transport [GO:0015878], GO:0015880, thiamine transport [GO:0015888], glutathione transport [GO:0034635], GO:0042918, GO:0046963, thioester transport [GO:1901337], glucosinolate transport [GO:1901349], sulfate transmembrane transport [GO:1902358], GO:1902558, sulfathiazole transmembrane transport [GO:1902599] Also known as: sulfur-containing compound transport Sources: GOC:mah Definition: The directed movement of compounds that contain sulfur, out of or within a cell, or between cells, by means of some agent such as a transporter or pore. Relationships: is a type of transport [GO:0006810]